regulation of zoospore formation [GO:0075240] (biological process) Sources: GOC:pamgo_curators Subtypes: positive regulation of zoospore formation [GO:0075241], negative regulation of zoospore formation [GO:0075242] Relationships: is a type of regulation of sporangiospore formation [GO:0075286]; regulates zoospore formation [GO:0075239] Definition: Any process that modulates the frequency, rate or extent of zoospore formation, a process in which a diploid cell undergoes meiosis, and the meiotic products acquire specialized features of asexual motile mononucleate flagellated spores called zoospores.